transition between fast and slow fiber [GO:0014883] (biological process) Sources: GOC:ef, GOC:mtg_muscle Definition: The process of conversion of fast-contracting muscle fibers to a slower character. This may involve slowing of contractile rate, slow myosin gene induction, increase in oxidative metabolic properties, altered electrophysiology and altered innervation. This process also regulates skeletal muscle adapatation. Also known as: transition between fast and slow fibre, transition fast-slow fiber, transition fast-slow fibre Relationships: is a type of regulation of skeletal muscle adaptation [GO:0014733]